D-lactate dehydrogenase (FAD) activity [GO:0140170] (molecular function) Relationships: is a type of D-lactate dehydrogenase activity [GO:0047809] Sources: RHEA:82479 Definition: Catalysis of the reaction: (R)-lactate + FAD + H+ = FADH2 + pyruvate.